regulation of glucocorticoid metabolic process [GO:0031943] (biological process) Also known as: regulation of glucocorticoid metabolism Relationships: is a type of GO:0019218; is a type of regulation of hormone metabolic process [GO:0032350]; regulates glucocorticoid metabolic process [GO:0008211] Definition: Any process that modulates the frequency, rate or extent of the chemical reactions and pathways involving glucocorticoids. Sources: GOC:mah Subtypes: GO:0031946, GO:0031949